{
  "gene": "UniProtKB:Q8NI38",
  "term_label": "nucleus",
  "gene_symbol": "NFKBID",
  "gene_name": "NF-kappa-B inhibitor delta",
  "term_id": "GO:0005634"
}